molybdopterin-synthase sulfurtransferase activity [GO:0061604] (molecular function) Relationships: is a type of GO:0016783 References: PMID:18154309, PMID:22370186 Sources: EC:2.8.1.11, GOC:dph Definition: Catalysis of the reaction: [Molybdopterin-synthase sulfur-carrier protein]-Gly-Gly-AMP + [cysteine desulfurase]-S-sulfanyl-L-cysteine = AMP [molybdopterin-synthase sulfur-carrier protein]-Gly-NH-CH(2)-C(O)SH + cysteine desulfurase.